{
  "term_id": "UNKNOWN:0001",
  "gene_symbol": "ZNF428",
  "term_label": "Unknown molecular function",
  "gene": "UniProtKB:Q96B54",
  "gene_name": "Zinc finger protein 428"
}